{
  "gene": "UniProtKB:Q9P2E5",
  "gene_symbol": "CHPF2",
  "term_label": "chondroitin sulfate proteoglycan biosynthetic process",
  "term_id": "GO:0050650",
  "gene_name": "Chondroitin sulfate glucuronyltransferase"
}